{
  "gene_symbol": "GFPT2",
  "gene": "UniProtKB:O94808",
  "term_label": "protein N-linked glycosylation",
  "term_id": "GO:0006487",
  "gene_name": "Glutamine--fructose-6-phosphate aminotransferase [isomerizing] 2"
}